{
  "term_label": "endoplasmic reticulum membrane",
  "term_id": "GO:0005789",
  "gene": "UniProtKB:Q96HY6",
  "gene_symbol": "DDRGK1",
  "gene_name": "DDRGK domain-containing protein 1"
}